{
  "gene": "UniProtKB:Q14568",
  "gene_name": "Heat shock protein HSP 90-alpha A2",
  "term_label": "protein-containing complex",
  "term_id": "GO:0032991",
  "gene_symbol": "HSP90AA2P"
}